{
  "term_id": "UNKNOWN:0001",
  "gene_symbol": "PDZD4",
  "gene": "UniProtKB:Q76G19",
  "term_label": "Unknown molecular function",
  "gene_name": "PDZ domain-containing protein 4"
}